{
  "term_label": "nucleus",
  "term_id": "GO:0005634",
  "gene_symbol": "MT1A",
  "gene": "UniProtKB:P04731",
  "gene_name": "Metallothionein-1A"
}